angiotensin-activated signaling pathway [GO:0038166] (biological process) Definition: A G protein-coupled receptor signaling pathway initiated by angiotensin II binding to its receptor on the surface of a target cell, and ending with the regulation of a downstream cellular process, e.g. transcription. References: PMID:10977869 Sources: GOC:BHF, GOC:mtg_cardiac_conduct_nov11, GOC:nhn, GOC:signaling Relationships: is_a G protein-coupled receptor signaling pathway [GO:0007186]; is part of GO:1904385 Subtypes: phospholipase C-activating angiotensin-activated signaling pathway [GO:0086097], GO:0086098 Regulation: regulated by regulation of angiotensin-activated signaling pathway [GO:0110061]; negatively regulated by negative regulation of angiotensin-activated signaling pathway [GO:0110062]; positively regulated by positive regulation of angiotensin-activated signaling pathway [GO:0110063] Also known as: angiotensin II-mediated signaling pathway, angiotensin receptor signaling pathway, angiotensin-mediated signaling pathway